{
  "term_id": "GO:0060271",
  "gene_symbol": "IFT46",
  "gene": "UniProtKB:Q9NQC8",
  "gene_name": "Intraflagellar transport protein 46 homolog",
  "term_label": "cilium assembly"
}